gentamycin catabolic process [GO:1901129] (biological process) Also known as: gentamycin breakdown, gentamycin catabolism, gentamycin degradation Relationships: is a type of aminoglycoside antibiotic catabolic process [GO:0030649]; is a type of polyol catabolic process [GO:0046174]; is a type of gentamycin metabolic process [GO:1901128] Definition: The chemical reactions and pathways resulting in the breakdown of gentamycin. Sources: GOC:TermGenie, GOC:yaf, UniPathway:UPA00967